{
  "gene": "UniProtKB:Q9NPJ6",
  "term_id": "GO:0070847",
  "gene_name": "Mediator of RNA polymerase II transcription subunit 4",
  "term_label": "core mediator complex",
  "gene_symbol": "MED4"
}